{
  "gene": "UniProtKB:P10163",
  "gene_name": "Basic salivary proline-rich protein 4",
  "term_id": "UNKNOWN:0001",
  "term_label": "Unknown molecular function",
  "gene_symbol": "PRB4"
}